{
  "gene_symbol": "ITLN1",
  "gene": "UniProtKB:Q8WWA0",
  "term_label": "oligosaccharide binding",
  "gene_name": "Intelectin-1",
  "term_id": "GO:0070492"
}